{
  "term_label": "plasma membrane",
  "gene_name": "Broad substrate specificity ATP-binding cassette transporter ABCG2",
  "gene": "UniProtKB:Q9UNQ0",
  "term_id": "GO:0005886",
  "gene_symbol": "ABCG2"
}